{
  "term_label": "ubiquitin protein ligase binding",
  "gene_symbol": "FATE1",
  "gene": "UniProtKB:Q969F0",
  "term_id": "GO:0031625",
  "gene_name": "Fetal and adult testis-expressed transcript protein"
}